corticospinal neuron axon guidance [GO:0021966] (biological process) Relationships: is a type of axon guidance [GO:0007411]; is part of corticospinal tract morphogenesis [GO:0021957] Definition: The process in which the migration of an axon growth cone of a neuron that is part of the corticospinal tract is directed from the cerebral cortex layer V to the spinal cord dorsal funiculus in response to a combination of attractive and repulsive cues. Also known as: corticospinal neuron axon pathfinding References: PMID:9878731 Sources: GOC:cls, GOC:dgh, GOC:dph, GOC:jid, GO_REF:0000021